{
  "gene_name": "Protein HEXIM1",
  "gene_symbol": "HEXIM1",
  "term_id": "GO:0004861",
  "term_label": "cyclin-dependent protein serine/threonine kinase inhibitor activity",
  "gene": "UniProtKB:O94992"
}